enzyme regulator activity [GO:0030234] (molecular function) Definition: A molecular function regulator that modulates a catalytic activity. Sources: GOC:pdt Also known as: catalytic regulator activity, enzyme modulator, metalloenzyme regulator activity Note: This term should only be used in cases when the regulator directly interacts with the enzyme, but does not result in a covalent modification. Relationships: is a type of molecular function regulator activity [GO:0098772]; regulates catalytic activity [GO:0003824] Subtypes: GO:0004857, GO:0008047, cyclase regulator activity [GO:0010851], kinase regulator activity [GO:0019207], GO:0019208, nitric-oxide synthase regulator activity [GO:0030235], histone deacetylase regulator activity [GO:0035033], histone acetyltransferase regulator activity [GO:0035034], GO:0042349, ornithine decarboxylase regulator activity [GO:0042979], GO:0043028, UTP:glucose-1-phosphate uridylyltransferase regulator activity [GO:0043763], methionine adenosyltransferase regulator activity [GO:0048270], ligase regulator activity [GO:0055103], ubiquitin-protein transferase regulator activity [GO:0055106], GTP cyclohydrolase I regulator activity [GO:0060308], nucleoside-triphosphatase regulator activity [GO:0060589], peptidase regulator activity [GO:0061134], inositol phosphoceramide synthase regulator activity [GO:0070917], DNA topoisomerase type II (double strand cut, ATP-hydrolyzing) regulator activity [GO:0072586], dolichol-phosphate-mannose synthase regulator activity [GO:0097713], methyltransferase regulator activity [GO:0141107], acetolactate synthase regulator activity [GO:1990610]